positive regulation of inclusion body assembly [GO:0090261] (biological process) Sources: GOC:tb Subtypes: positive regulation of Lewy body formation [GO:0140124], positive regulation of neurofibrillary tangle assembly [GO:1902998] Relationships: is_a positive regulation of cellular component biogenesis [GO:0044089]; is a type of positive regulation of cellular component organization [GO:0051130]; is a type of regulation of inclusion body assembly [GO:0090083]; positively regulates inclusion body assembly [GO:0070841] Definition: Any process that increases the rate, frequency, or extent of inclusion body assembly. Inclusion body assembly is the aggregation, arrangement and bonding together of a set of components to form an inclusion body.